{
  "term_label": "Unknown cellular component",
  "gene_symbol": "FARP2",
  "term_id": "UNKNOWN:0003",
  "gene_name": "FERM, ARHGEF and pleckstrin domain-containing protein 2",
  "gene": "UniProtKB:O94887"
}